cytokinin-activated signaling pathway [GO:0009736] (biological process) References: PMID:24080474 Sources: GOC:sm Definition: The series of molecular signals generated by the binding of a cytokinin to a receptor, and ending with the regulation of a downstream cellular process, e.g. transcription. Relationships: is a type of hormone-mediated signaling pathway [GO:0009755]; is part of GO:0071368 Also known as: cytokinin mediated signalling, cytokinin signaling, cytokinin mediated signaling pathway Regulation: regulated by regulation of cytokinin-activated signaling pathway [GO:0080036]; negatively regulated by GO:0080037; positively regulated by positive regulation of cytokinin-activated signaling pathway [GO:0080038]